dCDP metabolic process [GO:0046062] (biological process) Definition: The chemical reactions and pathways involving dCDP, deoxycytidine 5'-diphosphate. Sources: GOC:go_curators Also known as: dCDP metabolism Relationships: is a type of pyrimidine deoxyribonucleoside diphosphate metabolic process [GO:0009196]; is a type of pyrimidine deoxyribonucleotide metabolic process [GO:0009219] Subtypes: dCDP biosynthetic process [GO:0006240], dCDP catabolic process [GO:0006251]